{
  "term_id": "UNKNOWN:0003",
  "term_label": "Unknown cellular component",
  "gene_name": "Rho GTPase-activating protein 20",
  "gene_symbol": "ARHGAP20",
  "gene": "UniProtKB:Q9P2F6"
}